{
  "gene": "UniProtKB:Q8NCV1",
  "gene_name": "Adenosine deaminase domain-containing protein 2",
  "gene_symbol": "ADAD2",
  "term_id": "GO:0008251",
  "term_label": "tRNA-specific adenosine deaminase activity"
}